{
  "term_label": "Unknown biological process",
  "term_id": "UNKNOWN:0002",
  "gene_symbol": "CA14",
  "gene_name": "Carbonic anhydrase 14",
  "gene": "UniProtKB:Q9ULX7"
}